{
  "gene_symbol": "H2AC12",
  "term_label": "nucleosome",
  "gene_name": "Histone H2A type 1-H",
  "term_id": "GO:0000786",
  "gene": "UniProtKB:Q96KK5"
}